{
  "term_label": "protein folding in endoplasmic reticulum",
  "gene_symbol": "ERO1A",
  "term_id": "GO:0034975",
  "gene": "UniProtKB:Q96HE7",
  "gene_name": "ERO1-like protein alpha"
}